O-acetylhomoserine aminocarboxypropyltransferase activity [GO:0003961] (molecular function) Sources: EC:2.5.1.49 Subtypes: O-acetylhomoserine sulfhydrylase activity [GO:0051009] Relationships: is a type of transferase activity, transferring alkyl or aryl (other than methyl) groups [GO:0016765]; is part of 'de novo' L-methionine biosynthetic process [GO:0071266] Also known as: L-methionine anabolism, direct, from O-acetyl-L-homoserine, L-methionine biosynthetic process, direct, from O-acetyl-L-homoserine, L-methionine formation, direct, from O-acetyl-L-homoserine, L-methionine synthesis, direct, from O-acetyl-L-homoserine, O-acetylhomoserine (thiol)-lyase activity, methionine biosynthetic process, direct, from O-acetyl-L-homoserine, O-acetyl-L-homoserine acetate-lyase (adding methanethiol) activity, O-acetyl-L-homoserine sulfhydrolase activity, O-acetyl-L-homoserine:methanethiol 3-amino-3-carboxypropyltransferase activity, O-acetylhomoserine sulfhydrolase activity, OAH sulfhydrylase activity Definition: Catalysis of the reaction: O-acetyl-L-homoserine + methanethiol = L-methionine + acetate. Also reacts with other thiols and H2S, producing homocysteine or thioethers.